{
  "gene_symbol": "THTPA",
  "gene_name": "Thiamine-triphosphatase",
  "term_label": "Unknown cellular component",
  "term_id": "UNKNOWN:0003",
  "gene": "UniProtKB:Q9BU02"
}